{
  "gene_name": "Neuronal acetylcholine receptor subunit alpha-7",
  "term_label": "synapse",
  "gene": "UniProtKB:P36544",
  "term_id": "GO:0045202",
  "gene_symbol": "CHRNA7"
}